{
  "gene_symbol": "TRIM27",
  "term_id": "GO:0061630",
  "gene": "UniProtKB:P14373",
  "gene_name": "Zinc finger protein RFP",
  "term_label": "ubiquitin protein ligase activity"
}